{
  "gene_name": "Calcium-binding protein 2",
  "gene_symbol": "CABP2",
  "gene": "UniProtKB:Q9NPB3",
  "term_id": "GO:0007602",
  "term_label": "phototransduction"
}